{
  "gene_name": "Proline-rich protein 23C",
  "gene_symbol": "PRR23C",
  "term_id": "UNKNOWN:0002",
  "gene": "UniProtKB:Q6ZRP0",
  "term_label": "Unknown biological process"
}